{
  "gene_symbol": "SPDYE14",
  "gene_name": "Putative speedy protein E14",
  "term_id": "UNKNOWN:0003",
  "gene": "UniProtKB:P0DUD3",
  "term_label": "Unknown cellular component"
}